lactose catabolic process via tagatose-6-phosphate [GO:0019512] (biological process) Sources: GOC:go_curators Also known as: lactose breakdown via tagatose-6-phosphate, lactose degradation via tagatose-6-phosphate Definition: The chemical reactions and pathways resulting in the breakdown of lactose, via the intermediate tagatose-6-phosphate. Relationships: is a type of lactose catabolic process [GO:0005990]